{
  "gene": "UniProtKB:Q9BXT6",
  "gene_symbol": "MOV10L1",
  "gene_name": "RNA helicase Mov10l1",
  "term_label": "cytosol",
  "term_id": "GO:0005829"
}